{
  "gene_name": "Putative uncharacterized protein MGC39545",
  "term_label": "Unknown biological process",
  "gene": "UniProtKB:Q8IYB0",
  "term_id": "UNKNOWN:0002",
  "gene_symbol": "Q8IYB0"
}